{
  "term_label": "Unknown molecular function",
  "term_id": "UNKNOWN:0001",
  "gene_symbol": "MBLAC2",
  "gene_name": "Acyl-coenzyme A thioesterase MBLAC2",
  "gene": "UniProtKB:Q68D91"
}